regulation of substance P secretion, neurotransmission [GO:1904494] (biological process) References: PMID:15292051 Sources: GOC:TermGenie, GO_REF:0000058 Definition: Any process that modulates the frequency, rate or extent of substance P secretion, neurotransmission. Relationships: is a type of GO:0046928; is a type of regulation of substance P secretion [GO:1904458]; regulates GO:1990793 Subtypes: GO:1904495, positive regulation of substance P secretion, neurotransmission [GO:1904496]